{
  "gene_name": "Olfactory receptor 8I2",
  "gene": "UniProtKB:Q8N0Y5",
  "gene_symbol": "OR8I2",
  "term_id": "GO:0004984",
  "term_label": "olfactory receptor activity"
}